{
  "gene_symbol": "TRAJ36",
  "term_label": "Unknown molecular function",
  "gene": "UniProtKB:A0A087WU04",
  "gene_name": "T cell receptor alpha joining 36 (Fragment)",
  "term_id": "UNKNOWN:0001"
}